cholesterol homeostasis [GO:0042632] (BP) Also known as: positive regulation of cholesterol homeostasis, regulation of cholesterol homeostasis Relationships: is_a sterol homeostasis [GO:0055092] Sources: GOC:go_curators Definition: Any process involved in the maintenance of an internal steady state of cholesterol within an organism or cell.